{
  "gene": "UniProtKB:Q8IYM9",
  "gene_symbol": "TRIM22",
  "term_label": "regulation of gene expression",
  "gene_name": "E3 ubiquitin-protein ligase TRIM22",
  "term_id": "GO:0010468"
}